{
  "gene_symbol": "SLC27A4",
  "term_id": "GO:0001676",
  "term_label": "long-chain fatty acid metabolic process",
  "gene_name": "Long-chain fatty acid transport protein 4",
  "gene": "UniProtKB:Q6P1M0"
}